{
  "gene": "UniProtKB:Q8TE73",
  "term_id": "GO:0051959",
  "gene_name": "Dynein axonemal heavy chain 5",
  "term_label": "dynein light intermediate chain binding",
  "gene_symbol": "DNAH5"
}